{
  "gene": "UniProtKB:A0A1B0GTY4",
  "gene_symbol": "TEX50",
  "term_label": "Unknown biological process",
  "term_id": "UNKNOWN:0002",
  "gene_name": "Testis-expressed protein 50"
}